{
  "term_id": "GO:0005634",
  "gene_name": "Ubiquitin-conjugating enzyme E2 C",
  "gene": "UniProtKB:O00762",
  "term_label": "nucleus",
  "gene_symbol": "UBE2C"
}